{
  "gene_symbol": "GIMAP2",
  "gene": "UniProtKB:Q9UG22",
  "term_id": "GO:0005783",
  "gene_name": "GTPase IMAP family member 2",
  "term_label": "endoplasmic reticulum"
}